{
  "term_id": "GO:0030992",
  "gene": "UniProtKB:Q96LB3",
  "gene_name": "Intraflagellar transport protein 74 homolog",
  "term_label": "intraciliary transport particle B",
  "gene_symbol": "IFT74"
}